{
  "term_label": "mitochondrion",
  "gene": "UniProtKB:Q9BSK2",
  "gene_symbol": "SLC25A33",
  "gene_name": "Solute carrier family 25 member 33",
  "term_id": "GO:0005739"
}